{
  "term_label": "Unknown cellular component",
  "gene": "UniProtKB:Q15170",
  "term_id": "UNKNOWN:0003",
  "gene_name": "Transcription elongation factor A protein-like 1",
  "gene_symbol": "TCEAL1"
}